peripheral tolerance induction [GO:0002465] (biological process) Definition: Tolerance induction in the peripheral lymphoid tissues: blood, lymph nodes, spleen, and mucosal-associated lymphoid tissues. Sources: GOC:jal, GO_REF:0000022, ISBN:0781735149 Relationships: is a type of tolerance induction dependent upon immune response [GO:0002461] Subtypes: GO:0002413, peripheral B cell tolerance induction [GO:0002451], peripheral T cell tolerance induction [GO:0002458], peripheral tolerance induction to nonself antigen [GO:0002464], peripheral tolerance induction to self antigen [GO:0002466] Regulation: regulated by regulation of peripheral tolerance induction [GO:0002658]; negatively regulated by GO:0002659; positively regulated by positive regulation of peripheral tolerance induction [GO:0002660]